{
  "gene": "UniProtKB:Q9BZF9",
  "term_label": "cytosol",
  "gene_name": "Uveal autoantigen with coiled-coil domains and ankyrin repeats",
  "gene_symbol": "UACA",
  "term_id": "GO:0005829"
}